{
  "gene_symbol": "BIN1",
  "gene": "UniProtKB:O00499",
  "term_id": "UNKNOWN:0002",
  "gene_name": "Myc box-dependent-interacting protein 1",
  "term_label": "Unknown biological process"
}